D-amino acid transmembrane transporter activity [GO:0042943] (molecular function) Relationships: is a type of amino acid transmembrane transporter activity [GO:0015171]; is a type of GO:0046943; is part of D-amino acid transport [GO:0042940] Sources: GOC:jl, GOC:jsg, GOC:mah, GOC:mtg_transport, ISBN:0815340729 Definition: Enables the transfer of D-amino acids from one side of a membrane to the other. D-amino acids are the D-enantiomers of amino acids. Subtypes: ABC-type D-methionine transporter activity [GO:0033232], D-alanine transmembrane transporter activity [GO:0042944], D-serine transmembrane transporter activity [GO:0042945], D-aspartate transmembrane transporter activity [GO:0140010] Also known as: D-amino acid transporter activity